{
  "gene_name": "UBX domain-containing protein 11",
  "term_id": "UNKNOWN:0003",
  "gene": "UniProtKB:Q5T124",
  "gene_symbol": "UBXN11",
  "term_label": "Unknown cellular component"
}